chemotaxis [GO:0006935] (biological process) Relationships: is a type of taxis [GO:0042330]; BFO_0000050 response to chemical [GO:0042221] Regulation: regulated by regulation of chemotaxis [GO:0050920]; positively regulated by positive regulation of chemotaxis [GO:0050921]; negatively regulated by GO:0050922 Also known as: taxis in response to chemical stimulus Subtypes: aerotaxis [GO:0009454], GO:0009455, GO:0034670, chemotaxis to oxidizable substrate [GO:0042333], chemotaxis to folate [GO:0043326], GO:0043327, positive chemotaxis [GO:0050918], negative chemotaxis [GO:0050919], cell chemotaxis [GO:0060326] Sources: ISBN:0198506732 Definition: The directed movement of a motile cell or organism, or the directed growth of a cell guided by a specific chemical concentration gradient. Movement may be towards a higher concentration (positive chemotaxis) or towards a lower concentration (negative chemotaxis).